{
  "gene_name": "Negative regulator of P-body association",
  "gene_symbol": "NBDY",
  "term_label": "P-body",
  "gene": "UniProtKB:A0A0U1RRE5",
  "term_id": "GO:0000932"
}